{
  "gene_name": "Piwi-like protein 3",
  "term_label": "piRNA binding",
  "term_id": "GO:0034584",
  "gene_symbol": "PIWIL3",
  "gene": "UniProtKB:Q7Z3Z3"
}